{
  "gene": "UniProtKB:A8MV24",
  "term_label": "Unknown biological process",
  "term_id": "UNKNOWN:0002",
  "gene_name": "Uncharacterized protein C17orf98",
  "gene_symbol": "C17orf98"
}